{
  "gene_symbol": "TRMT61A",
  "gene_name": "tRNA (adenine(58)-N(1))-methyltransferase catalytic subunit TRMT61A",
  "term_label": "tRNA (adenine(58)-N1)-methyltransferase activity",
  "term_id": "GO:0160107",
  "gene": "UniProtKB:Q96FX7"
}